{
  "gene": "UniProtKB:P22059",
  "term_id": "GO:0032934",
  "gene_symbol": "OSBP",
  "term_label": "sterol binding",
  "gene_name": "Oxysterol-binding protein 1"
}